negative regulation of granzyme A production [GO:2000512] (biological process) Relationships: is_a negative regulation of production of molecular mediator of immune response [GO:0002701]; is a type of GO:2000511; negatively regulates granzyme A production [GO:0035746] Definition: Any process that stops, prevents or reduces the frequency, rate or extent of granzyme A production. Sources: GOC:obol